{
  "gene_name": "GA-binding protein subunit beta-2",
  "gene_symbol": "GABPB2",
  "term_label": "nucleus",
  "term_id": "GO:0005634",
  "gene": "UniProtKB:Q8TAK5"
}